{
  "gene": "UniProtKB:P06396",
  "gene_symbol": "GSN",
  "term_label": "actin polymerization or depolymerization",
  "gene_name": "Gelsolin",
  "term_id": "GO:0008154"
}